glycerophosphoinositol inositolphosphodiesterase activity [GO:0047394] (molecular function) Relationships: is_a phosphoric diester hydrolase activity [GO:0008081] Definition: Catalysis of the reaction: H2O + 1-(sn-glycero-3-phospho)-1D-myoinositol = 1D-myo-inositol 1-phosphate + glycerol. Sources: EC:3.1.4.43, MetaCyc:3.1.4.43-RXN Also known as: 1,2-cyclic-inositol-phosphate phosphodiesterase activity, 1-(sn-glycero-3-phospho)-1D-myo-inositol inositolphosphohydrolase activity, 1-D-myo-inositol-1,2-cyclic-phosphate 2-inositolphosphohydrolase activity, D-inositol 1,2-cyclic phosphate 2-phosphohydrolase activity, D-myo-inositol 1,2-cyclic phosphate 2-phosphohydrolase activity, D-myo-inositol 1:2-cyclic phosphate 2-phosphohydrolase activity, inositol-1,2-cyclic-phosphate 2-inositolphosphohydrolase activity